{
  "gene_name": "Vomeronasal type-1 receptor 5",
  "gene": "UniProtKB:Q7Z5H4",
  "gene_symbol": "VN1R5",
  "term_id": "UNKNOWN:0002",
  "term_label": "Unknown biological process"
}